{
  "term_label": "nucleoplasm",
  "term_id": "GO:0005654",
  "gene_symbol": "PML",
  "gene_name": "Protein PML",
  "gene": "UniProtKB:P29590"
}